{
  "gene": "UniProtKB:Q8IWF9",
  "gene_symbol": "CCDC83",
  "term_label": "Unknown molecular function",
  "term_id": "UNKNOWN:0001",
  "gene_name": "Coiled-coil domain-containing protein 83"
}